{
  "term_id": "UNKNOWN:0001",
  "gene": "UniProtKB:Q8N660",
  "gene_name": "Neuroblastoma breakpoint family member 15",
  "term_label": "Unknown molecular function",
  "gene_symbol": "NBPF15"
}